{
  "gene_name": "FSD1-like protein",
  "term_label": "Unknown molecular function",
  "gene_symbol": "FSD1L",
  "term_id": "UNKNOWN:0001",
  "gene": "UniProtKB:Q9BXM9"
}